{
  "gene_name": "Solute carrier family 25 member 34",
  "gene": "UniProtKB:Q6PIV7",
  "gene_symbol": "SLC25A34",
  "term_id": "UNKNOWN:0002",
  "term_label": "Unknown biological process"
}